positive gravitaxis [GO:0048061] (biological process) Also known as: positive geotactic behavior, positive geotactic behaviour, positive gravitactic behavior, positive gravitactic behaviour, positive taxis in response to gravity, positive taxis in response to gravitytaxis in response to gravitational stimulus Relationships: is a type of gravitaxis [GO:0042332] Sources: GOC:jid Definition: The directed movement of a motile cell or organism towards the source of gravity.